DNA endonuclease activity, producing 3'-phosphomonoesters [GO:0016889] (molecular function) Relationships: is a type of DNA endonuclease activity [GO:0004520]; is a type of hydrolase activity, acting on ester bonds [GO:0016788] Definition: Catalysis of the hydrolysis of ester linkages within deoxyribonucleic acids by creating internal breaks to yield 3'-phosphomonoesters. Also known as: endodeoxyribonuclease activity, producing 3'-phosphomonoesters, endodeoxyribonuclease activity, producing other than 5'-phosphomonoesters Subtypes: deoxyribonuclease II activity [GO:0004531], crossover junction DNA endonuclease activity [GO:0008821], GO:0048257 Sources: GOC:ai